{
  "term_id": "GO:0003723",
  "term_label": "RNA binding",
  "gene_name": "Heterogeneous nuclear ribonucleoprotein C-like 1",
  "gene": "UniProtKB:O60812",
  "gene_symbol": "HNRNPCL1"
}